{
  "gene": "UniProtKB:Q9Y2H9",
  "gene_name": "Microtubule-associated serine_threonine-protein kinase 1",
  "gene_symbol": "MAST1",
  "term_label": "microtubule cytoskeleton",
  "term_id": "GO:0015630"
}